isopentenyl diphosphate biosynthetic process, methylerythritol 4-phosphate pathway involved in terpenoid biosynthetic process [GO:0051484] (biological process) Also known as: isopentenyl diphosphate anabolism, mevalonate-independent pathway, during terpenoid anabolism, isopentenyl diphosphate biosynthetic process, mevalonate-independent pathway involved in terpenoid biosynthetic process, isopentenyl diphosphate biosynthetic process, mevalonate-independent pathway, during terpenoid biosynthetic process, isopentenyl diphosphate formation, mevalonate-independent pathway, during terpenoid biosynthesis, isopentenyl diphosphate formation, mevalonate-independent pathway, during terpenoid formation, isopentenyl diphosphate synthesis, mevalonate-independent pathway, during terpenoid synthesis Definition: The chemical reactions and pathways resulting in the formation of isopentenyl diphosphate by the mevalonate-independent pathway that contributes to terpenoid biosynthesis. Isopentenyl diphosphate (IPP) is the fundamental unit in isoprenoid biosynthesis and is biosynthesized from pyruvate and glyceraldehyde 3-phosphate via intermediates, including 1-deoxy-D-xylulose 5-phosphate. Sources: GOC:ai Relationships: is a type of isopentenyl diphosphate biosynthetic process, methylerythritol 4-phosphate pathway [GO:0019288]; BFO_0000050 terpenoid biosynthetic process, mevalonate-independent [GO:0051483]